{
  "gene_symbol": "MIR17HG",
  "term_label": "Unknown biological process",
  "gene": "UniProtKB:Q75NE6",
  "term_id": "UNKNOWN:0002",
  "gene_name": "Putative microRNA 17 host gene protein"
}